{
  "gene_name": "Protein FAM186B",
  "gene": "UniProtKB:Q8IYM0",
  "term_id": "UNKNOWN:0003",
  "term_label": "Unknown cellular component",
  "gene_symbol": "FAM186B"
}